primary miRNA processing [GO:0031053] (biological process) Definition: A process involved in the conversion of a primary microRNA transcript into a pre-microRNA molecule. Relationships: is a type of miRNA processing [GO:0035196] Also known as: pri-miRNA processing, primary miRNA modification, primary microRNA processing, primary miRNA methylation Regulation: RO_0002211 by regulation of primary miRNA processing [GO:2000634]; negatively regulated by negative regulation of primary miRNA processing [GO:2000635]; positively regulated by positive regulation of primary miRNA processing [GO:2000636] References: PMID:15211354, PMID:25799998 Sources: GOC:sl